{
  "gene": "UniProtKB:Q92629",
  "gene_symbol": "SGCD",
  "term_id": "GO:0048738",
  "gene_name": "Delta-sarcoglycan",
  "term_label": "cardiac muscle tissue development"
}